{
  "term_label": "Unknown biological process",
  "gene_symbol": "HIPK4",
  "gene": "UniProtKB:Q8NE63",
  "term_id": "UNKNOWN:0002",
  "gene_name": "Homeodomain-interacting protein kinase 4"
}